phenanthrol glycosyltransferase activity [GO:0019112] (molecular function) Definition: Catalysis of the reaction: phenanthrol + glucose = phenanthryl-beta-D-glucopyranoside + H2O. Relationships: is a type of GO:0016758 Sources: GOC:ai